{
  "term_id": "GO:0005783",
  "gene_symbol": "ATP2C2",
  "gene_name": "Calcium-transporting ATPase type 2C member 2",
  "gene": "UniProtKB:O75185",
  "term_label": "endoplasmic reticulum"
}